{
  "gene_symbol": "GNAO1",
  "term_label": "G-protein beta/gamma-subunit complex binding",
  "gene_name": "Guanine nucleotide-binding protein G(o) subunit alpha",
  "gene": "UniProtKB:P09471",
  "term_id": "GO:0031683"
}